osmiophilic body [GO:0044310] (cellular component) Definition: A membrane-bounded vesicle found predominantly in Plasmodium female gametocytes, that becomes progressively more abundant as the gametocyte reaches full maturity. These vesicles lie beneath the subpellicular membrane of the gametocyte, and the release of their contents into the parasitophorous vacuole has been postulated to aid in the escape of gametocytes from the erythrocyte after ingestion by the mosquito. References: PMID:18086189 Sources: GOC:jl Relationships: is a type of cytoplasmic vesicle [GO:0031410]